{
  "gene": "UniProtKB:A6NIN4",
  "term_label": "protein ubiquitination",
  "term_id": "GO:0016567",
  "gene_symbol": "RNF227",
  "gene_name": "RING finger protein 227"
}